{
  "gene_name": "Spindle and centriole-associated protein 1",
  "term_id": "GO:0090307",
  "gene_symbol": "SPICE1",
  "term_label": "mitotic spindle assembly",
  "gene": "UniProtKB:Q8N0Z3"
}